{
  "gene": "UniProtKB:A6NJ78",
  "gene_symbol": "METTL15",
  "gene_name": "12S rRNA N4-methylcytidine (m4C) methyltransferase",
  "term_id": "UNKNOWN:0003",
  "term_label": "Unknown cellular component"
}